negative regulation of epithelial cell apoptotic process [GO:1904036] (biological process) Also known as: down regulation of epithelial cell apoptotic process, down regulation of epitheliocyte apoptotic process, down-regulation of epithelial cell apoptotic process, down-regulation of epitheliocyte apoptotic process, downregulation of epithelial cell apoptotic process, downregulation of epitheliocyte apoptotic process, negative regulation of epitheliocyte apoptotic process, down regulation of epithelial cell apoptosis, down regulation of epitheliocyte apoptosis, down-regulation of epithelial cell apoptosis, down-regulation of epitheliocyte apoptosis, downregulation of epithelial cell apoptosis, downregulation of epitheliocyte apoptosis, inhibition of epithelial cell apoptosis, inhibition of epithelial cell apoptotic process, inhibition of epitheliocyte apoptosis, inhibition of epitheliocyte apoptotic process, negative regulation of epithelial cell apoptosis, negative regulation of epitheliocyte apoptosis Subtypes: GO:1902173, negative regulation of hepatocyte apoptotic process [GO:1903944], GO:1904193, negative regulation of podocyte apoptotic process [GO:1904634], negative regulation of granulosa cell apoptotic process [GO:1904709], negative regulation of type B pancreatic cell apoptotic process [GO:2000675] Definition: Any process that stops, prevents or reduces the frequency, rate or extent of epithelial cell apoptotic process. Relationships: is a type of negative regulation of apoptotic process [GO:0043066]; is a type of regulation of epithelial cell apoptotic process [GO:1904035]; negatively regulates epithelial cell apoptotic process [GO:1904019] References: PMID:19137015 Sources: GOC:TermGenie, GO_REF:0000058